bicellular tight junction assembly [GO:0070830] (biological process) Regulation: negatively regulated by negative regulation of bicellular tight junction assembly [GO:1903347]; positively regulated by positive regulation of bicellular tight junction assembly [GO:1903348]; regulated by regulation of bicellular tight junction assembly [GO:2000810] Definition: The aggregation, arrangement and bonding together of a set of components to form a tight junction, an occluding cell-cell junction that is composed of a branching network of sealing strands that completely encircles the apical end of each cell in an epithelial sheet. Relationships: is a type of tight junction assembly [GO:0120192]; is part of apical junction assembly [GO:0043297] Sources: GOC:mah Also known as: tight junction formation